{
  "gene": "UniProtKB:P41247",
  "gene_symbol": "PNPLA4",
  "gene_name": "Patatin-like phospholipase domain-containing protein 4",
  "term_label": "cytoplasm",
  "term_id": "GO:0005737"
}